positive regulation of B cell antigen processing and presentation [GO:0002624] (biological process) Definition: Any process that activates or increases the frequency, rate, or extent of B cell antigen processing and presentation. Sources: GOC:add Also known as: positive regulation of B lymphocyte antigen processing and presentation, positive regulation of B-cell antigen processing and presentation, positive regulation of B-lymphocyte antigen processing and presentation, up regulation of B cell antigen processing and presentation, up-regulation of B cell antigen processing and presentation, upregulation of B cell antigen processing and presentation, activation of B cell antigen processing and presentation, stimulation of B cell antigen processing and presentation Relationships: is_a positive regulation of antigen processing and presentation [GO:0002579]; is a type of regulation of B cell antigen processing and presentation [GO:0002622]; positively regulates B cell antigen processing and presentation [GO:0002450]